{
  "gene_name": "Zinc finger protein 791",
  "gene_symbol": "ZNF791",
  "gene": "UniProtKB:Q3KP31",
  "term_id": "GO:0005634",
  "term_label": "nucleus"
}